alpha-L-fucosidase activity [GO:0004560] (molecular function) Relationships: is_a fucosidase activity [GO:0015928] Sources: EC:3.2.1.51 Also known as: alpha-L-fucoside fucohydrolase activity, alpha-fucosidase activity Subtypes: GO:0033932, 1,6-alpha-L-fucosidase activity [GO:0033938], 1,2-alpha-L-fucosidase activity [GO:0047513] Definition: Catalysis of the reaction: an alpha-L-fucoside + H2O = an alcohol + L-fucose.